{
  "gene_name": "Iroquois-class homeodomain protein IRX-3",
  "term_id": "GO:0048468",
  "gene": "UniProtKB:P78415",
  "term_label": "cell development",
  "gene_symbol": "IRX3"
}